{
  "gene": "UniProtKB:A4D161",
  "term_label": "Unknown molecular function",
  "gene_name": "Protein FAM221A",
  "term_id": "UNKNOWN:0001",
  "gene_symbol": "FAM221A"
}